{
  "gene_symbol": "CLPP",
  "gene": "UniProtKB:Q16740",
  "gene_name": "ATP-dependent Clp protease proteolytic subunit, mitochondrial",
  "term_label": "protein quality control for misfolded or incompletely synthesized proteins",
  "term_id": "GO:0006515"
}